{
  "gene_name": "Insulin-like growth factor 2 mRNA-binding protein 3",
  "gene_symbol": "IGF2BP3",
  "term_id": "GO:0010494",
  "term_label": "cytoplasmic stress granule",
  "gene": "UniProtKB:O00425"
}